sodium ion transmembrane transporter activity [GO:0015081] (molecular function) Also known as: sodium transporter activity Subtypes: GO:0005272, GO:0005432, P-type sodium transporter activity [GO:0008554], solute:sodium symporter activity [GO:0015370], sodium:proton antiporter activity [GO:0015385], sodium ion uniporter activity [GO:0022818], tetrahydromethanopterin S-methyltransferase activity [GO:0030269], sodium-transporting ATP synthase activity, rotational mechanism [GO:0046932], sodium-transporting ATPase activity, rotational mechanism [GO:0046962], magnesium:sodium antiporter activity [GO:0061768], ABC-type sodium transporter activity [GO:0140679], GO:0140892 Relationships: is a type of GO:0046873; is part of sodium ion transmembrane transport [GO:0035725] Definition: Enables the transfer of sodium ions (Na+) from one side of a membrane to the other. Sources: GOC:BHF, GOC:ai Regulation: regulated by regulation of sodium ion transmembrane transporter activity [GO:2000649]; positively regulated by GO:2000651